{
  "gene_name": "Cyclic nucleotide-gated cation channel alpha-4",
  "term_id": "GO:0005886",
  "gene_symbol": "CNGA4",
  "gene": "UniProtKB:Q8IV77",
  "term_label": "plasma membrane"
}